nerve growth factor receptor binding [GO:0005163] (molecular function) Also known as: NGF receptor binding, nerve growth factor receptor ligand, neurotrophin Definition: Binding to a nerve growth factor receptor. References: PMID:15654015 Sources: GOC:ai Relationships: is a type of GO:0005123; is_a neurotrophin receptor binding [GO:0005165]